{
  "term_id": "GO:0005829",
  "gene_symbol": "PPP2R2B",
  "term_label": "cytosol",
  "gene": "UniProtKB:Q00005",
  "gene_name": "Serine_threonine-protein phosphatase 2A 55 kDa regulatory subunit B beta isoform"
}